{
  "gene": "UniProtKB:O95965",
  "term_label": "integrin complex",
  "term_id": "GO:0008305",
  "gene_symbol": "ITGBL1",
  "gene_name": "Integrin beta-like protein 1"
}